{
  "term_id": "GO:0072659",
  "gene": "UniProtKB:O60894",
  "gene_symbol": "RAMP1",
  "term_label": "protein localization to plasma membrane",
  "gene_name": "Receptor activity-modifying protein 1"
}